nitrate reductase complex [GO:0009325] (cellular component) Definition: An enzyme complex that catalyzes the formation of nitrate from nitrite with the concomitant reduction of an acceptor. Subtypes: NarGHI complex [GO:0044799] Relationships: is a type of GO:1990204 References: PMID:2139607